{
  "gene": "UniProtKB:Q15915",
  "term_id": "GO:0000981",
  "gene_name": "Zinc finger protein ZIC 1",
  "term_label": "DNA-binding transcription factor activity, RNA polymerase II-specific",
  "gene_symbol": "ZIC1"
}